{
  "term_id": "GO:0005737",
  "gene_symbol": "MTMR8",
  "term_label": "cytoplasm",
  "gene_name": "Myotubularin-related protein 8",
  "gene": "UniProtKB:Q96EF0"
}